{
  "term_id": "GO:1903078",
  "gene_name": "SH3 and cysteine-rich domain-containing protein 3",
  "gene_symbol": "STAC3",
  "term_label": "positive regulation of protein localization to plasma membrane",
  "gene": "UniProtKB:Q96MF2"
}